{
  "term_label": "structural constituent of muscle",
  "gene_name": "Myosin-binding protein C, cardiac-type",
  "gene_symbol": "MYBPC3",
  "gene": "UniProtKB:Q14896",
  "term_id": "GO:0008307"
}